{
  "gene": "UniProtKB:Q8WU17",
  "gene_symbol": "RNF139",
  "term_id": "GO:0036503",
  "term_label": "ERAD pathway",
  "gene_name": "E3 ubiquitin-protein ligase RNF139"
}